{
  "gene_symbol": "TUBA8",
  "gene_name": "Tubulin alpha-8 chain",
  "gene": "UniProtKB:Q9NY65",
  "term_label": "microtubule",
  "term_id": "GO:0005874"
}